{
  "gene": "UniProtKB:Q08AD1",
  "gene_name": "Calmodulin-regulated spectrin-associated protein 2",
  "term_label": "cytoplasmic microtubule organization",
  "gene_symbol": "CAMSAP2",
  "term_id": "GO:0031122"
}